{
  "gene_name": "GDNF family receptor alpha-like",
  "gene": "UniProtKB:Q6UXV0",
  "term_label": "nervous system development",
  "gene_symbol": "GFRAL",
  "term_id": "GO:0007399"
}